{
  "gene": "UniProtKB:Q7Z442",
  "gene_name": "Polycystin-1-like protein 2",
  "term_label": "detection of mechanical stimulus",
  "term_id": "GO:0050982",
  "gene_symbol": "PKD1L2"
}